{
  "term_id": "GO:0005737",
  "gene_name": "Peptidyl-prolyl cis-trans isomerase A-like 4F",
  "term_label": "cytoplasm",
  "gene": "UniProtKB:P0DN26",
  "gene_symbol": "PPIAL4F"
}